{
  "gene": "UniProtKB:O95070",
  "term_id": "GO:0030134",
  "gene_name": "Protein YIF1A",
  "gene_symbol": "YIF1A",
  "term_label": "COPII-coated ER to Golgi transport vesicle"
}